{
  "gene_symbol": "CDK1",
  "gene_name": "Cyclin-dependent kinase 1",
  "term_id": "GO:0005634",
  "term_label": "nucleus",
  "gene": "UniProtKB:P06493"
}